paraferritin complex [GO:0070826] (cellular component) Relationships: is a type of protein-containing complex [GO:0032991]; is part of cytoplasm [GO:0005737] Definition: A cytoplasmic protein complex that contains integrin, mobilferrin and a flavin monooxygenase, is capable of reducing Fe(III) to Fe(II) utilizing NADPH, and is involved in iron transport. Fe(II) is required in the cell as the substrate for ferrochelatase in the synthesis of heme. References: PMID:11842004, PMID:8639593 Sources: GOC:mah, GOC:rph